{
  "term_id": "GO:0005737",
  "term_label": "cytoplasm",
  "gene_name": "Tubulin--tyrosine ligase-like protein 12",
  "gene_symbol": "TTLL12",
  "gene": "UniProtKB:Q14166"
}